{
  "gene": "UniProtKB:Q5JTZ9",
  "gene_name": "Alanine--tRNA ligase, mitochondrial",
  "term_label": "mitochondrion",
  "gene_symbol": "AARS2",
  "term_id": "GO:0005739"
}